 [IAO:0000589]